{
  "gene": "UniProtKB:Q6P1K2",
  "term_id": "GO:0000444",
  "gene_symbol": "PMF1",
  "gene_name": "Polyamine-modulated factor 1",
  "term_label": "MIS12/MIND type complex"
}